{
  "gene": "UniProtKB:Q8N9U9",
  "gene_name": "Putative uncharacterized protein SPANXA2-OT1",
  "gene_symbol": "SPANXA2-OT1",
  "term_id": "UNKNOWN:0003",
  "term_label": "Unknown cellular component"
}